{
  "gene": "UniProtKB:Q6N063",
  "gene_name": "2-oxoglutarate and iron-dependent oxygenase domain-containing protein 2",
  "term_id": "UNKNOWN:0003",
  "term_label": "Unknown cellular component",
  "gene_symbol": "OGFOD2"
}